{
  "gene_symbol": "ZNF92",
  "term_label": "DNA-binding transcription factor activity, RNA polymerase II-specific",
  "gene_name": "Zinc finger protein 92",
  "term_id": "GO:0000981",
  "gene": "UniProtKB:Q03936"
}